{
  "term_id": "GO:0006953",
  "gene_symbol": "APCS",
  "term_label": "acute-phase response",
  "gene_name": "Serum amyloid P-component",
  "gene": "UniProtKB:P02743"
}